{
  "gene_symbol": "PFDN5",
  "gene": "UniProtKB:Q99471",
  "gene_name": "Prefoldin subunit 5",
  "term_id": "UNKNOWN:0001",
  "term_label": "Unknown molecular function"
}